{
  "gene_symbol": "DCTN1",
  "gene": "UniProtKB:Q14203",
  "gene_name": "Dynactin subunit 1",
  "term_label": "spindle pole",
  "term_id": "GO:0000922"
}